{
  "gene": "UniProtKB:P26373",
  "gene_name": "Large ribosomal subunit protein eL13",
  "term_id": "UNKNOWN:0002",
  "term_label": "Unknown biological process",
  "gene_symbol": "RPL13"
}